{
  "term_id": "GO:0001228",
  "gene_symbol": "UBP1",
  "term_label": "DNA-binding transcription activator activity, RNA polymerase II-specific",
  "gene": "UniProtKB:Q9NZI7",
  "gene_name": "Upstream-binding protein 1"
}